{
  "term_id": "GO:0045095",
  "gene_name": "Keratin, type I cytoskeletal 19",
  "gene": "UniProtKB:P08727",
  "term_label": "keratin filament",
  "gene_symbol": "KRT19"
}